{
  "term_label": "Unknown molecular function",
  "term_id": "UNKNOWN:0001",
  "gene_symbol": "CLCA3P",
  "gene_name": "Calcium-activated chloride channel regulator family member 3",
  "gene": "UniProtKB:Q9Y6N3"
}